{
  "gene_name": "Cathepsin S",
  "term_id": "GO:0005615",
  "term_label": "extracellular space",
  "gene": "UniProtKB:P25774",
  "gene_symbol": "CTSS"
}